tri-(feruloyl or hydroxyferuloyl) spermidine meta-hydroxylase activity [GO:0072532] (molecular function) Definition: Catalysis of the meta-hydroxylation of any of the three phenolic rings on triferuloyl spermidine or any of its mono- or di-(hydroxyferuloyl)-spermidine derivatives. Note: Note that the overall reaction representing three successive executions of this activity is N1,N5,N10-triferuloyl spermidine + 3 NADPH + 3 O2 = N1,N5,N10-tri-(hydroxyferuloyl)-spermidine + 3 NADP+ + 3 H2O; this corresponds to the MetaCyc reaction RXN-11262 (http://biocyc.org/META/NEW-IMAGE?type=REACTION&object=RXN-11262) and the KEGG reaction R08986 (http://www.genome.jp/dbget-bin/www_bget?rn:R08986). References: PMID:19779199 Sources: GOC:kad Subtypes: triferuloylspermidine meta-hydroxylase activity [GO:0072550], diferuloyl mono-(hydroxyferuloyl) spermidine meta-hydroxylase activity [GO:0072551], monoferuloyl di-(hydroxyferuloyl) spermidine meta-hydroxylase activity [GO:0072552] Relationships: is a type of oxidoreductase activity, acting on paired donors, with incorporation or reduction of molecular oxygen, NAD(P)H as one donor, and incorporation of one atom of oxygen [GO:0016709]